{
  "gene_symbol": "ADGRL1",
  "gene_name": "Adhesion G protein-coupled receptor L1",
  "gene": "UniProtKB:O94910",
  "term_label": "latrotoxin receptor activity",
  "term_id": "GO:0016524"
}